{
  "gene": "UniProtKB:P20585",
  "gene_name": "DNA mismatch repair protein Msh3",
  "term_id": "GO:0016447",
  "term_label": "somatic recombination of immunoglobulin gene segments",
  "gene_symbol": "MSH3"
}